L-valine catabolic process to isobutanol [GO:1902697] (biological process) References: PMID:9748245 Sources: GOC:TermGenie, GOC:mengo_curators, GO_REF:0000093 Also known as: valine breakdown to isobutanol, valine catabolism to isobutanol, valine degradation to isobutanol Definition: The chemical reactions and pathways resulting in the breakdown of L-valine to isobutanol. Relationships: is a type of GO:0006574; is a type of primary alcohol metabolic process [GO:0034308]